{
  "term_label": "positive regulation of osteoclast differentiation",
  "term_id": "GO:0045672",
  "gene_symbol": "TNFSF11",
  "gene_name": "Tumor necrosis factor ligand superfamily member 11",
  "gene": "UniProtKB:O14788"
}